{
  "gene_symbol": "ATG9B",
  "gene_name": "Autophagy-related protein 9B",
  "gene": "UniProtKB:Q674R7",
  "term_id": "GO:0005776",
  "term_label": "autophagosome"
}